DNA beta-glucosyltransferase activity [GO:0033821] (molecular function) Also known as: T4 phage beta-glucosyltransferase activity, T4-HMC-beta-glucosyl transferase activity, T4-beta-glucosyl transferase activity, UDP glucose-DNA beta-glucosyltransferase activity, UDP-glucose:DNA beta-D-glucosyltransferase activity, UDPglucose:DNA beta-D-glucosyltransferase activity, uridine diphosphoglucose-deoxyribonucleate beta-glucosyltransferase activity Relationships: is a type of glucosyltransferase activity [GO:0046527]; is a type of catalytic activity, acting on DNA [GO:0140097] Sources: EC:2.4.1.27 Definition: Catalysis of the transfer of a beta-D-glucosyl residue from UDP-glucose to a hydroxymethylcytosine residue in DNA.